{
  "gene_name": "Zinc finger protein 337",
  "gene_symbol": "ZNF337",
  "term_label": "RNA polymerase II transcription regulatory region sequence-specific DNA binding",
  "term_id": "GO:0000977",
  "gene": "UniProtKB:Q9Y3M9"
}